{
  "term_label": "cellular response to glucose starvation",
  "term_id": "GO:0042149",
  "gene": "UniProtKB:O43159",
  "gene_symbol": "RRP8",
  "gene_name": "Ribosomal RNA-processing protein 8"
}